clavaminate synthase activity [GO:0033758] (molecular function) Sources: EC:1.14.11.21 Definition: Catalysis of the reactions: deoxyamidinoproclavaminate + 2-oxoglutarate + O2 = amidinoproclavaminate + succinate + CO2 + H2O; proclavaminate + 2-oxoglutarate + O2 = dihydroclavaminate + succinate + CO2 + 2 H2O; and dihydroclavaminate + 2-oxoglutarate + O2 = clavaminate + succinate + CO2 + 2 H2O. Also known as: clavaminate synthase 2 activity, clavaminic acid synthase activity, deoxyamidinoproclavaminate,2-oxoglutarate:oxygen oxidoreductase (3-hydroxylating) activity Relationships: is a type of 2-oxoglutarate-dependent dioxygenase activity [GO:0016706]